{
  "term_label": "phosphoribosylaminoimidazolesuccinocarboxamide synthase activity",
  "gene": "UniProtKB:P22234",
  "gene_symbol": "PAICS",
  "term_id": "GO:0004639",
  "gene_name": "Bifunctional phosphoribosylaminoimidazole carboxylase_phosphoribosylaminoimidazole succinocarboxamide synthetase"
}